cholest-4-en-3-one 26-monooxygenase activity [GO:0036199] (molecular function) Sources: EC:1.14.15.29 Relationships: is a type of oxidoreductase activity, acting on paired donors, with incorporation or reduction of molecular oxygen, NAD(P)H as one donor, and incorporation of one atom of oxygen [GO:0016709] Definition: Catalysis of the reaction: cholest-4-en-3-one + NADH + H+ + O2 = 26-hydroxycholest-4-en-3-one + NAD+ + H2O. This reaction involves the hydroxylation of the C26 carbon, followed by oxidation of the alcohol to the carboxylic acid via the aldehyde intermediate.